{
  "gene_symbol": "IL31RA",
  "gene": "UniProtKB:Q8NI17",
  "term_label": "cytokine receptor activity",
  "gene_name": "Interleukin-31 receptor subunit alpha",
  "term_id": "GO:0004896"
}